positive regulation of intrinsic apoptotic signaling pathway in response to osmotic stress by p53 class mediator [GO:1902240] (biological process) Definition: Any process that activates or increases the frequency, rate or extent of intrinsic apoptotic signaling pathway in response to osmotic stress by p53 class mediator. References: PMID:16571598 Sources: GOC:TermGenie, GOC:krc, GOC:mtg_apoptosis Also known as: up regulation of intrinsic apoptotic signaling pathway in response to osmotic stress by p53 class mediator, up-regulation of intrinsic apoptotic signaling pathway in response to osmotic stress by p53 class mediator, upregulation of intrinsic apoptotic signaling pathway in response to osmotic stress by p53 class mediator, activation of intrinsic apoptotic signaling pathway in response to osmotic stress by p53 class mediator Relationships: is a type of positive regulation of intrinsic apoptotic signaling pathway in response to osmotic stress [GO:1902220]; is a type of regulation of intrinsic apoptotic signaling pathway in response to osmotic stress by p53 class mediator [GO:1902238]; is_a positive regulation of intrinsic apoptotic signaling pathway by p53 class mediator [GO:1902255]; positively regulates intrinsic apoptotic signaling pathway in response to osmotic stress by p53 class mediator [GO:1990127]